PUMA-BCL-2 complex [GO:0097142] (cellular component) References: PMID:14634621 Sources: GOC:so Definition: A heterodimeric protein complex consisting of PUMA and BCL-2, members of the Bcl-2 family of anti- and proapoptotic regulators. Relationships: is a type of Bcl-2 family protein complex [GO:0097136]